{
  "gene_symbol": "ASCL1",
  "gene_name": "Achaete-scute homolog 1",
  "gene": "UniProtKB:P50553",
  "term_id": "GO:0045944",
  "term_label": "positive regulation of transcription by RNA polymerase II"
}